{
  "term_label": "Unknown molecular function",
  "gene": "UniProtKB:A0A0B4J277",
  "gene_name": "T cell receptor alpha variable 22",
  "term_id": "UNKNOWN:0001",
  "gene_symbol": "TRAV22"
}